{
  "gene_symbol": "TMEM181",
  "gene_name": "Transmembrane protein 181",
  "gene": "UniProtKB:Q9P2C4",
  "term_id": "UNKNOWN:0002",
  "term_label": "Unknown biological process"
}